{
  "term_id": "UNKNOWN:0001",
  "gene_name": "PWWP domain-containing DNA repair factor 3B",
  "gene": "UniProtKB:Q5H9M0",
  "term_label": "Unknown molecular function",
  "gene_symbol": "PWWP3B"
}